{
  "gene_name": "HMG box-containing protein 1",
  "gene": "UniProtKB:O60381",
  "gene_symbol": "HBP1",
  "term_id": "GO:0005634",
  "term_label": "nucleus"
}